{
  "term_id": "GO:0003713",
  "gene_name": "Activating signal cointegrator 1",
  "term_label": "transcription coactivator activity",
  "gene": "UniProtKB:Q15650",
  "gene_symbol": "TRIP4"
}